{
  "gene_name": "Two pore channel protein 1",
  "gene": "UniProtKB:Q9ULQ1",
  "term_label": "lysosomal membrane",
  "term_id": "GO:0005765",
  "gene_symbol": "TPCN1"
}